{
  "gene_name": "Tubulin beta 8B",
  "gene_symbol": "TUBB8B",
  "gene": "UniProtKB:A6NNZ2",
  "term_label": "GTP binding",
  "term_id": "GO:0005525"
}